negative regulation of photoreceptor cell differentiation [GO:0046533] (biological process) Sources: GOC:go_curators Definition: Any process that stops, prevents, or reduces the frequency, rate or extent of photoreceptor cell differentiation. An example of this process is found in Drosophila melanogaster. Relationships: is a type of negative regulation of neuron differentiation [GO:0045665]; is a type of regulation of photoreceptor cell differentiation [GO:0046532]; is a type of negative regulation of multicellular organismal process [GO:0051241]; RO_0002212 photoreceptor cell differentiation [GO:0046530] Also known as: down regulation of photoreceptor cell differentiation, down regulation of photoreceptor differentiation, down-regulation of photoreceptor cell differentiation, down-regulation of photoreceptor differentiation, downregulation of photoreceptor cell differentiation, downregulation of photoreceptor differentiation, negative regulation of photoreceptor differentiation, inhibition of photoreceptor cell differentiation, inhibition of photoreceptor differentiation Subtypes: negative regulation of retinal cone cell fate commitment [GO:0060226], negative regulation of compound eye photoreceptor cell differentiation [GO:0110118]